{
  "gene_name": "Nuclear protein localization protein 4 homolog",
  "term_id": "GO:0006511",
  "gene": "UniProtKB:Q8TAT6",
  "term_label": "ubiquitin-dependent protein catabolic process",
  "gene_symbol": "NPLOC4"
}